oxidoreductase activity, acting on hydrogen as donor, with other known acceptors [GO:0046995] (molecular function) Definition: Catalysis of an oxidation-reduction (redox) reaction in which hydrogen reduces a known acceptor other than a cytochrome, an iron-sulfur protein, NAD, NADP, or a quinone or similar compound. Sources: GOC:ai Relationships: is a type of oxidoreductase activity, acting on hydrogen as donor [GO:0016695] Subtypes: GO:0033796, GO:0047068, GO:0050454, Methanosarcina-phenazine hydrogenase activity [GO:0051911]